{
  "term_label": "immunoglobulin mediated immune response",
  "gene_symbol": "IGHV1-2",
  "gene": "UniProtKB:P23083",
  "gene_name": "Immunoglobulin heavy variable 1-2",
  "term_id": "GO:0016064"
}